{
  "gene": "UniProtKB:P37268",
  "term_id": "GO:0006695",
  "gene_symbol": "FDFT1",
  "gene_name": "Squalene synthase",
  "term_label": "cholesterol biosynthetic process"
}